{
  "gene_name": "Histone acetyltransferase KAT6A",
  "term_label": "chromatin",
  "term_id": "GO:0000785",
  "gene_symbol": "KAT6A",
  "gene": "UniProtKB:Q92794"
}